very long-chain fatty acid metabolic process [GO:0000038] (BP) Definition: The chemical reactions and pathways involving a very long-chain fatty acid. A very long-chain fatty acid has an aliphatic tail containing more than 22 carbons. Relationships: is a type of fatty acid metabolic process [GO:0006631] Subtypes: GO:0042760, very long-chain fatty acid biosynthetic process [GO:0042761] Note: While there is not universal consensus on the lengths of short-, medium-, long- and very-long-chain fatty acids, the GO uses the definitions in ChEBI (see CHEBI:26666, CHEBI:59554, CHEBI:15904 and CHEBI:27283). Sources: GOC:hjd Also known as: very long chain fatty acid metabolic process, very-long-chain fatty acid metabolic process, very-long-chain fatty acid metabolism